{
  "term_id": "GO:2000051",
  "gene": "UniProtKB:Q63HN8",
  "gene_symbol": "RNF213",
  "gene_name": "E3 ubiquitin-protein ligase RNF213",
  "term_label": "negative regulation of non-canonical Wnt signaling pathway"
}